{
  "gene_symbol": "FGF9",
  "term_id": "GO:0005615",
  "term_label": "extracellular space",
  "gene_name": "Fibroblast growth factor 9",
  "gene": "UniProtKB:P31371"
}